{
  "gene_name": "Extracellular superoxide dismutase [Cu-Zn]",
  "gene": "UniProtKB:P08294",
  "term_id": "UNKNOWN:0003",
  "gene_symbol": "SOD3",
  "term_label": "Unknown cellular component"
}